{
  "gene_name": "Zinc finger protein 605",
  "term_label": "Unknown molecular function",
  "term_id": "UNKNOWN:0001",
  "gene": "UniProtKB:Q86T29",
  "gene_symbol": "ZNF605"
}